protein localization to perinuclear region of cytoplasm [GO:1905719] (biological process) Definition: A process in which a protein is transported to, or maintained in, a location within the perinuclear region of the cytoplasm. References: PMID:15177031 Sources: GOC:TermGenie, GO_REF:0000087 Also known as: protein localisation in perinuclear region of cytoplasm, protein localisation to perinuclear region of cytoplasm, protein localization in perinuclear region of cytoplasm, protein localization to perinuclear cytoplasm Relationships: is a type of GO:0008104